ornithine decarboxylase regulator activity [GO:0042979] (molecular function) Subtypes: ornithine decarboxylase inhibitor activity [GO:0008073], GO:0042978 Relationships: is a type of GO:0030234; regulates GO:0004586 Sources: GOC:jl Definition: Binds to and modulates the activity of the enzyme ornithine decarboxylase.